{
  "term_id": "GO:0031012",
  "term_label": "extracellular matrix",
  "gene_name": "Collectin-12",
  "gene": "UniProtKB:Q5KU26",
  "gene_symbol": "COLEC12"
}